{
  "gene_name": "SPRY domain-containing protein 3",
  "term_label": "Unknown cellular component",
  "gene_symbol": "SPRYD3",
  "gene": "UniProtKB:Q8NCJ5",
  "term_id": "UNKNOWN:0003"
}